{
  "term_id": "GO:0000792",
  "term_label": "heterochromatin",
  "gene": "UniProtKB:Q9UK61",
  "gene_symbol": "TASOR",
  "gene_name": "Protein TASOR"
}